right horn of sinus venosus development [GO:0061080] (biological process) Definition: The progression of the right horn of the sinus venosus from its formation to the mature structure. Sources: GOC:dph Relationships: is a type of anatomical structure development [GO:0048856]; is part of sinus venosus development [GO:0003235]